{
  "gene": "UniProtKB:Q7Z4H4",
  "term_id": "GO:0003073",
  "gene_name": "Protein ADM2",
  "term_label": "regulation of systemic arterial blood pressure",
  "gene_symbol": "ADM2"
}